transmembrane signaling receptor activity [GO:0004888] (MF) Definition: Combining with an extracellular or intracellular signal and transmitting the signal from one side of the membrane to the other to initiate a change in cell activity or state as part of signal transduction. Relationships: is a type of GO:0038023 Sources: GOC:go_curators, Wikipedia:Transmembrane_receptor Note: This term includes intracellular membrane receptors, e.g. IP3 triggered release of Ca2+ from intracellular stores. Subtypes: GO:0001571, opsonin receptor activity [GO:0001847], complement receptor activity [GO:0004875], GO:0004896, G protein-coupled receptor activity [GO:0004930], olfactory receptor activity [GO:0004984], osmosensor activity [GO:0005034], death receptor activity [GO:0005035], netrin receptor activity [GO:0005042], GO:0005056, GO:0008046, GO:0008066, hedgehog receptor activity [GO:0008158], sulfonylurea receptor activity [GO:0008281], taste receptor activity [GO:0008527], cytokinin receptor activity [GO:0009884], acetylcholine receptor activity [GO:0015464], nucleotide receptor activity [GO:0016502], latrotoxin receptor activity [GO:0016524], GABA receptor activity [GO:0016917], semaphorin receptor activity [GO:0017154], GO:0019198, transmembrane receptor protein kinase activity [GO:0019199], immunoglobulin receptor activity [GO:0019763], ICAM-3 receptor activity [GO:0030369], GO:0030379, MHC class I receptor activity [GO:0032393], MHC class Ib receptor activity [GO:0032394], MHC class II receptor activity [GO:0032395], apolipoprotein A-I receptor activity [GO:0034188], reelin receptor activity [GO:0038025], collagen receptor activity [GO:0038064], neuregulin receptor activity [GO:0038131], Wnt receptor activity [GO:0042813], GO:0099589, GO:0140897 Also known as: transmembrane receptor activity, transmembrane signalling receptor activity